{
  "gene_symbol": "MRPL41",
  "gene_name": "Large ribosomal subunit protein mL41",
  "term_id": "GO:0003735",
  "gene": "UniProtKB:Q8IXM3",
  "term_label": "structural constituent of ribosome"
}